{
  "term_id": "GO:0006890",
  "gene": "UniProtKB:Q9H4A6",
  "gene_name": "Golgi phosphoprotein 3",
  "term_label": "retrograde vesicle-mediated transport, Golgi to endoplasmic reticulum",
  "gene_symbol": "GOLPH3"
}